regulation of mesonephric glomerular mesangial cell proliferation [GO:2000090] (biological process) Definition: Any process that modulates the frequency, rate or extent of mesonephric glomerular mesangial cell proliferation. Relationships: is a type of regulation of glomerular mesangial cell proliferation [GO:0072124]; is a type of regulation of cell proliferation involved in mesonephros development [GO:2000606]; regulates GO:0061269 Subtypes: negative regulation of mesonephric glomerular mesangial cell proliferation [GO:2000091], positive regulation of mesonephric glomerular mesangial cell proliferation [GO:2000092] Sources: GOC:mtg_kidney_jan10